{
  "gene_name": "Motor neuron and pancreas homeobox protein 1",
  "gene_symbol": "MNX1",
  "gene": "UniProtKB:P50219",
  "term_label": "sequence-specific double-stranded DNA binding",
  "term_id": "GO:1990837"
}